{
  "gene_symbol": "RABL6",
  "term_label": "Unknown biological process",
  "gene": "UniProtKB:Q3YEC7",
  "gene_name": "Rab-like protein 6",
  "term_id": "UNKNOWN:0002"
}